site of DNA damage [GO:0090734] (cellular component) Definition: A region of a chromosome at which DNA damage has occurred. DNA damage signaling and repair proteins accumulate at the lesion to respond to the damage and repair the DNA to form a continuous DNA helix. Relationships: is a type of cellular anatomical structure [GO:0110165]; is part of chromosome [GO:0005694] Sources: GOC:pg Subtypes: site of double-strand break [GO:0035861]